{
  "gene": "UniProtKB:P41162",
  "term_id": "GO:0000981",
  "term_label": "DNA-binding transcription factor activity, RNA polymerase II-specific",
  "gene_name": "ETS translocation variant 3",
  "gene_symbol": "ETV3"
}